{
  "gene_symbol": "SNX27",
  "gene_name": "Sorting nexin-27",
  "gene": "UniProtKB:Q96L92",
  "term_id": "GO:0005769",
  "term_label": "early endosome"
}